annealing activity [GO:0140666] (molecular function) Also known as: renaturation Subtypes: RNA strand annealing activity [GO:0033592], GO:0097098, DNA/DNA annealing activity [GO:1990814] Relationships: is a type of nucleic acid binding [GO:0003676]; is a type of nucleic acid conformation isomerase activity [GO:0120545]; is a type of catalytic activity, acting on a nucleic acid [GO:0140640] References: PMID:22888405 Definition: An activity that facilitates the formation of a complementary double-stranded polynucleotide molecule.